uracil import across plasma membrane [GO:0098721] (biological process) Also known as: uracil import into cell Regulation: RO_0002211 by regulation of uracil import across plasma membrane [GO:1905529]; negatively regulated by negative regulation of uracil import across plasma membrane [GO:1905530]; positively regulated by positive regulation of uracil import across plasma membrane [GO:1905531] Definition: The directed movement of uracil from outside of a cell, across the plasma membrane and into the cytosol. Relationships: is a type of import across plasma membrane [GO:0098739]; is a type of uracil transmembrane transport [GO:1903791] Sources: GOC:dos